{
  "gene_symbol": "PNKP",
  "gene_name": "Bifunctional polynucleotide phosphatase_kinase",
  "term_label": "DNA repair",
  "gene": "UniProtKB:Q96T60",
  "term_id": "GO:0006281"
}